{
  "gene": "UniProtKB:O00231",
  "gene_name": "26S proteasome non-ATPase regulatory subunit 11",
  "term_label": "proteasome regulatory particle, lid subcomplex",
  "gene_symbol": "PSMD11",
  "term_id": "GO:0008541"
}